{
  "term_label": "Unknown cellular component",
  "gene_name": "Radial spoke head 10 homolog B",
  "gene": "UniProtKB:P0C881",
  "term_id": "UNKNOWN:0003",
  "gene_symbol": "RSPH10B"
}